{
  "gene_name": "Fibrous sheath-interacting protein 1",
  "gene_symbol": "FSIP1",
  "term_id": "UNKNOWN:0002",
  "gene": "UniProtKB:Q8NA03",
  "term_label": "Unknown biological process"
}